synaptic transmission, dopaminergic [GO:0001963] (biological process) Relationships: is a type of chemical synaptic transmission [GO:0007268] Definition: The vesicular release of dopamine. from a presynapse, across a chemical synapse, the subsequent activation of dopamine receptors at the postsynapse of a target cell (neuron, muscle, or secretory cell) and the effects of this activation on the postsynaptic membrane potential and ionic composition of the postsynaptic cytosol. This process encompasses both spontaneous and evoked release of neurotransmitter and all parts of synaptic vesicle exocytosis. Evoked transmission starts with the arrival of an action potential at the presynapse. Regulation: regulated by regulation of synaptic transmission, dopaminergic [GO:0032225]; positively regulated by GO:0032226; negatively regulated by negative regulation of synaptic transmission, dopaminergic [GO:0032227] Sources: GOC:dos, GOC:dph Also known as: dopaminergic synaptic transmission